{
  "term_label": "DNA-binding transcription factor activity, RNA polymerase II-specific",
  "gene_name": "Zinc finger protein 426",
  "gene": "UniProtKB:Q9BUY5",
  "term_id": "GO:0000981",
  "gene_symbol": "ZNF426"
}